{
  "gene": "UniProtKB:Q15393",
  "term_id": "GO:0000398",
  "gene_name": "Splicing factor 3B subunit 3",
  "gene_symbol": "SF3B3",
  "term_label": "mRNA splicing, via spliceosome"
}